{
  "gene_symbol": "BPIFA1",
  "term_label": "surfactant homeostasis",
  "term_id": "GO:0043129",
  "gene_name": "BPI fold-containing family A member 1",
  "gene": "UniProtKB:Q9NP55"
}